negative regulation of secretion of lysosomal enzymes [GO:0090341] (biological process) Definition: Any process that decreases the rate, frequency or extent of secretion of lysosomal enzymes, the controlled release of lysosomal enzymes by a cell. Relationships: is a type of negative regulation of protein secretion [GO:0050709]; is a type of GO:0090182; negatively regulates secretion of lysosomal enzymes [GO:0033299] Sources: GOC:BHF